{
  "term_id": "UNKNOWN:0003",
  "gene": "UniProtKB:A1A4V9",
  "gene_name": "Cilia- and flagella-associated protein 119",
  "gene_symbol": "CFAP119",
  "term_label": "Unknown cellular component"
}